mesangial cell development [GO:0072143] (biological process) Relationships: is_a GO:0048468; is part of GO:0072007 Definition: The process whose specific outcome is the progression of a mesangial cell in the kidney over time, from its formation to the mature structure. Sources: GOC:mtg_kidney_jan10 Subtypes: glomerular mesangial cell development [GO:0072144]